{
  "gene_symbol": "MUC21",
  "gene_name": "Mucin-21",
  "gene": "UniProtKB:A0A0G2JKD1",
  "term_id": "UNKNOWN:0002",
  "term_label": "Unknown biological process"
}